{
  "term_label": "cytosol",
  "term_id": "GO:0005829",
  "gene_symbol": "AKR1B15",
  "gene_name": "Aldo-keto reductase family 1 member B15",
  "gene": "UniProtKB:C9JRZ8"
}